{
  "term_label": "protein serine/threonine kinase activator activity",
  "gene_symbol": "TPX2",
  "term_id": "GO:0043539",
  "gene": "UniProtKB:Q9ULW0",
  "gene_name": "Targeting protein for Xklp2"
}